{
  "gene": "UniProtKB:P67775",
  "term_label": "cytosol",
  "gene_symbol": "PPP2CA",
  "gene_name": "Serine_threonine-protein phosphatase 2A catalytic subunit alpha isoform",
  "term_id": "GO:0005829"
}